regulation of red or far-red light signaling pathway [GO:0090227] (biological process) Subtypes: positive regulation of red or far-red light signaling pathway [GO:0090228], negative regulation of red or far-red light signaling pathway [GO:0090229] Relationships: is a type of regulation of signal transduction [GO:0009966]; is a type of GO:2000030; regulates red or far-red light signaling pathway [GO:0010017] Definition: Any process that modulates the rate, frequency or extent of the red or far-red signaling pathway, the series of molecular signals initiated upon sensing by photoreceptor molecules of red light or far red light. Also known as: regulation of phytochrome signaling pathway, regulation of red or far-red light signalling pathway Sources: GOC:tb